thymocyte aggregation [GO:0071594] (biological process) Also known as: immature T cell aggregation, immature T-cell aggregation, T cell precursor aggregation, immature T-lymphocyte aggregation, thymic lymphocyte aggregation References: PMID:1382990 Sources: GOC:sl Relationships: is a type of GO:0070489 Regulation: regulated by regulation of thymocyte aggregation [GO:2000398]; negatively regulated by GO:2000399; positively regulated by positive regulation of thymocyte aggregation [GO:2000400] Definition: The adhesion of one thymocyte (an immature T cell) to one or more other thymocytes via adhesion molecules.